glycine import into mitochondrion [GO:1904983] (biological process) Definition: The process in which glycine is transported from the cytosol into the mitochondrial matrix. References: PMID:26821380 Sources: GOC:TermGenie, GO_REF:0000078 Also known as: transmembrane glycine transport from cytosol to mitochondrion Relationships: is a type of amino acid transmembrane transport [GO:0003333]; is a type of GO:0015816; is a type of import into the mitochondrion [GO:0170036]; is a type of carboxylic acid transmembrane transport [GO:1905039]